cardioblast cell fate specification [GO:0042685] (biological process) Definition: The process in which a cell becomes capable of differentiating autonomously into a cardioblast cell in an environment that is neutral with respect to the developmental pathway; upon specification, the cell fate can be reversed. A cardioblast is a cardiac precursor cell. It is a cell that has been committed to a cardiac fate, but will undergo more cell division rather than terminally differentiating. Regulation: negatively regulated by negative regulation of cardioblast cell fate specification [GO:0009997]; regulated by regulation of cardioblast cell fate specification [GO:0042686] Relationships: is a type of cardiac cell fate specification [GO:0060912]; is part of GO:0042684 Sources: GOC:go_curators